{
  "term_id": "UNKNOWN:0002",
  "term_label": "Unknown biological process",
  "gene_name": "C-type lectin domain family 2 member L",
  "gene_symbol": "CLEC2L",
  "gene": "UniProtKB:P0C7M8"
}